{
  "gene_symbol": "RGPD3",
  "term_id": "GO:0005643",
  "gene_name": "RanBP2-like and GRIP domain-containing protein 3",
  "gene": "UniProtKB:A6NKT7",
  "term_label": "nuclear pore"
}